{
  "gene_symbol": "HSPA1A",
  "gene_name": "Heat shock 70 kDa protein 1A",
  "term_id": "GO:0042026",
  "term_label": "protein refolding",
  "gene": "UniProtKB:P0DMV8"
}